{
  "gene_name": "Interleukin-1 receptor accessory protein",
  "gene_symbol": "IL1RAP",
  "term_label": "cytokine-mediated signaling pathway",
  "gene": "UniProtKB:Q9NPH3",
  "term_id": "GO:0019221"
}